ubiquitin-like modifier activating enzyme activity [GO:0008641] (molecular function) Relationships: is a type of ligase activity, forming carbon-sulfur bonds [GO:0016877]; is a type of catalytic activity, acting on a protein [GO:0140096]; is a type of GO:0140657 Sources: GOC:jl, GOC:mah Subtypes: GO:0004839, Atg12 activating enzyme activity [GO:0019778], Atg8 activating enzyme activity [GO:0019779], FAT10 activating enzyme activity [GO:0019780], NEDD8 activating enzyme activity [GO:0019781], ISG15 activating enzyme activity [GO:0019782], SUMO activating enzyme activity [GO:0019948], URM1 activating enzyme activity [GO:0042292], Hub1 activating enzyme activity [GO:0042293], UFM1 activating enzyme activity [GO:0071566] Also known as: small protein activating enzyme activity Definition: Catalysis of the activation of small proteins, such as ubiquitin or ubiquitin-like proteins, through the formation of an ATP-dependent high-energy thiolester bond.